{
  "term_id": "GO:0043235",
  "gene_symbol": "RAMP1",
  "gene": "UniProtKB:O60894",
  "term_label": "receptor complex",
  "gene_name": "Receptor activity-modifying protein 1"
}